nephric duct morphogenesis [GO:0072178] (biological process) Subtypes: pronephric duct morphogenesis [GO:0039023], mesonephric duct morphogenesis [GO:0072180] Definition: The process in which the anatomical structures of the nephric duct are generated and organized. A nephric duct is a tube that drains a primitive kidney. Relationships: is a type of epithelial tube morphogenesis [GO:0060562]; BFO_0000050 nephric duct development [GO:0072176] Sources: GOC:mtg_kidney_jan10